U2-type catalytic step 1 spliceosome [GO:0071006] (cellular component) References: PMID:18322460, PMID:19239890 Sources: GOC:ab, GOC:krc, GOC:mah, ISBN:0879695897, ISBN:0879697393 Also known as: U2-type activated spliceosome, major catalytic step 1 spliceosome, GT-AG catalytic step 1 spliceosome, mammalian U2-type spliceosomal complex B*, mammalian U2-type spliceosomal complex B2, yeast U2-type spliceosomal complex A1 Relationships: is a type of U2-type spliceosomal complex [GO:0005684]; is a type of catalytic step 1 spliceosome [GO:0071012]; has part U2 snRNP [GO:0005686]; has part U6 snRNP [GO:0005688] Definition: A spliceosomal complex that is formed by the displacement of the U1 and U4 snRNPs from the precatalytic spliceosome; the U2, U5 and U6 snRNPs remain associated with the mRNA. This complex, sometimes called the activated spliceosome, is the catalytically active form of the spliceosome, and includes many proteins in addition to those found in the U2, and U5 and U6 snRNPs.